{
  "term_label": "Unknown molecular function",
  "gene": "UniProtKB:Q5VYM1",
  "term_id": "UNKNOWN:0001",
  "gene_name": "Uncharacterized protein C9orf131",
  "gene_symbol": "C9orf131"
}